{
  "gene_name": "Olfactory receptor 4B1",
  "term_id": "GO:0005886",
  "gene": "UniProtKB:Q8NGF8",
  "gene_symbol": "OR4B1",
  "term_label": "plasma membrane"
}